{
  "gene": "UniProtKB:Q9BQ51",
  "gene_name": "Programmed cell death 1 ligand 2",
  "term_label": "external side of plasma membrane",
  "gene_symbol": "PDCD1LG2",
  "term_id": "GO:0009897"
}